{
  "gene_name": "Trafficking protein particle complex subunit 11",
  "term_label": "Unknown cellular component",
  "gene_symbol": "TRAPPC11",
  "gene": "UniProtKB:Q7Z392",
  "term_id": "UNKNOWN:0003"
}